ATP-dependent activity [GO:0140657] (molecular function) References: PMID:24878343, PMID:25750732, PMID:32933017, PMID:33818025, PMID:33873056, PMID:33988324 Definition: A molecular function characterized by the coupling of ATP hydrolysis to other steps of a reaction mechanism to make the reaction energetically favorable, for example to catalyze a reaction or drive transport against a concentration gradient. Subtypes: microfilament motor activity [GO:0000146], microtubule motor activity [GO:0003777], ATP-dependent peptidase activity [GO:0004176], helicase activity [GO:0004386], ATP-dependent activity, acting on DNA [GO:0008094], ATP-dependent activity, acting on RNA [GO:0008186], microtubule severing ATPase activity [GO:0008568], GO:0008641, fatty acid ligase activity [GO:0015645], calcium-dependent ATPase activity [GO:0030899], GO:0036402, ATPase-coupled transmembrane transporter activity [GO:0042626], tubulin-dependent ATPase activity [GO:0070463], ATPase-coupled intramembrane lipid transporter activity [GO:0140326], GO:0140545, membrane protein dislocase activity [GO:0140567], ATP-dependent protein folding chaperone [GO:0140662], ATP-dependent FeS chaperone activity [GO:0140663], GO:1990833 Relationships: is a type of molecular_function [GO:0003674]; has part ATP hydrolysis activity [GO:0016887] Note: Note that this term represents a grouping class that includes all proteins that use ATP hydrolysis to drive a reaction; it is not meant to capture the ATP hydrolysis reaction itself. To annotate ATP hydrolysis, please use 'ATP hydrolysis activity ; GO:0016887'. Regulation: positively regulated by ATPase activator activity [GO:0001671]; negatively regulated by GO:0032780; positively regulated by positive regulation of ATP-dependent activity [GO:0032781]; RO_0002212 by ATPase inhibitor activity [GO:0042030]; regulated by GO:0043462; regulated by ATPase regulator activity [GO:0060590] Also known as: ATP hydrolysis-dependent activity, ATPase activity, ATPase activity, coupled, ATPase-dependent activity